{
  "gene": "UniProtKB:A0A1B0GTD5",
  "gene_name": "Testis-expressed protein 49",
  "term_id": "UNKNOWN:0002",
  "gene_symbol": "SPMIP11",
  "term_label": "Unknown biological process"
}